Mis6-Sim4 complex [GO:0031511] (cellular component) Also known as: Mis6-Mal2-Sim4 centromere complex, Sim4 complex, Mis6 centromere subcomplex, Mcm21 Definition: A protein complex that forms part of the inner kinetochore, which is involved in the loading of the centromeric histone h3 variant CENP-A onto centromeres and in centromere specific heterochromatin formation. The complex contains about 12 proteins, of which two are known as Mis6 and Sim4 in S. pombe and CENP-I and CENP-H in human. Relationships: is a type of protein-containing complex [GO:0032991]; is part of inner kinetochore [GO:0000939] References: PMID:12719471, PMID:15897182 Sources: GOC:vw